{
  "gene_symbol": "MPV17L2",
  "gene_name": "Mpv17-like protein 2",
  "gene": "UniProtKB:Q567V2",
  "term_label": "cytoplasm",
  "term_id": "GO:0005737"
}